positive regulation of protein catabolic process [GO:0045732] (biological process) Sources: GOC:go_curators Also known as: positive regulation of cellular protein breakdown, positive regulation of cellular protein catabolic process, positive regulation of cellular protein catabolism, positive regulation of cellular protein degradation, positive regulation of protein breakdown, positive regulation of protein catabolism, positive regulation of protein degradation, up regulation of cellular protein breakdown, up regulation of cellular protein catabolic process, up regulation of cellular protein catabolism, up regulation of cellular protein degradation, up regulation of protein catabolic process, up-regulation of cellular protein breakdown, up-regulation of cellular protein catabolic process, up-regulation of cellular protein catabolism, up-regulation of cellular protein degradation, up-regulation of protein catabolic process, upregulation of cellular protein breakdown, upregulation of cellular protein catabolic process, upregulation of cellular protein catabolism, upregulation of cellular protein degradation, upregulation of protein catabolic process, activation of cellular protein breakdown, activation of cellular protein catabolic process, activation of cellular protein catabolism, activation of cellular protein degradation, activation of protein catabolic process, positive regulation of cyclin breakdown, positive regulation of cyclin catabolic process, positive regulation of cyclin catabolism, positive regulation of cyclin degradation, positive regulation of degradation of cyclin, stimulation of protein catabolic process Subtypes: positive regulation of proteolysis associated with antigen processing and presentation [GO:0002630], positive regulation of low-density lipoprotein particle receptor catabolic process [GO:0032805], positive regulation of membrane protein ectodomain proteolysis [GO:0051044], positive regulation of elastin catabolic process [GO:0110015], positive regulation of proteasomal protein catabolic process [GO:1901800], GO:1904352, positive regulation of chaperone-mediated autophagy [GO:1904716] Definition: Any process that activates or increases the frequency, rate or extent of the chemical reactions and pathways resulting in the breakdown of a protein by the destruction of the native, active configuration, with or without the hydrolysis of peptide bonds. Relationships: is a type of positive regulation of catabolic process [GO:0009896]; is a type of regulation of protein catabolic process [GO:0042176]; is a type of GO:0051247; positively regulates protein catabolic process [GO:0030163]